{
  "term_label": "nucleus",
  "term_id": "GO:0005634",
  "gene": "UniProtKB:Q99742",
  "gene_name": "Neuronal PAS domain-containing protein 1",
  "gene_symbol": "NPAS1"
}